regulation of initiation of premeiotic DNA replication [GO:1904512] (biological process) References: PMID:25891897 Sources: GOC:TermGenie, GO_REF:0000058 Also known as: regulation of premeiotic DNA replication initiation, regulation of initiation of meiotic DNA synthesis, regulation of initiation of premeiotic DNA synthesis, regulation of meiotic DNA replication initiation Subtypes: negative regulation of initiation of premeiotic DNA replication [GO:1904513], positive regulation of initiation of premeiotic DNA replication [GO:1904514] Definition: Any process that modulates the frequency, rate or extent of initiation of premeiotic DNA replication. Relationships: is a type of regulation of DNA-templated DNA replication initiation [GO:0030174]; is a type of regulation of nuclear cell cycle DNA replication [GO:0033262]; is a type of GO:0051445; regulates meiotic DNA replication initiation [GO:1902974]